hydroxymethylglutaryl-CoA reductase (NADPH) activity [GO:0004420] (molecular function) Definition: Catalysis of the reaction: (R)-mevalonate + CoA + 2 NADP+ = (S)-3-hydroxy-3-methylglutaryl-CoA + 2 H+ + 2 NADPH. References: PMID:29224355 Sources: RHEA:15989 Also known as: 3-hydroxy-3-methylglutaryl-coenzyme A reductase activity, HMG-CoA reductase activity, hydroxymethylglutaryl-CoA reductase activity Relationships: is a type of oxidoreductase activity, acting on the CH-OH group of donors, NAD or NADP as acceptor [GO:0016616]